{
  "gene_name": "RWD domain-containing protein 4",
  "term_id": "UNKNOWN:0002",
  "gene_symbol": "RWDD4",
  "gene": "UniProtKB:Q6NW29",
  "term_label": "Unknown biological process"
}